embryonic dorsal fin morphogenesis [GO:0035123] (biological process) Relationships: is a type of embryonic medial fin morphogenesis [GO:0035122]; is a type of GO:0035142 Definition: The process, occurring in the embryo, by which the anatomical structures of the dorsal fin are generated and organized. A dorsal fin is an unpaired medial fin on the dorsal aspect of a fish that provides lateral stability while swimming. Generally fish have one or two dorsal fins. Sources: GOC:dgh